{
  "gene_symbol": "DUXA",
  "term_id": "GO:0006357",
  "gene": "UniProtKB:A6NLW8",
  "gene_name": "Double homeobox protein A",
  "term_label": "regulation of transcription by RNA polymerase II"
}